sulfate adenylyltransferase complex (ATP) [GO:0009336] (cellular component) Relationships: is a type of adenylyltransferase complex [GO:1902503]; is part of GO:0005737 Definition: An enzyme complex that catalyzes the formation adenylylsulfate from sulfate and ATP. References: PMID:15184554 Also known as: sulphate adenylyltransferase complex (ATP)